negative regulation of tooth mineralization [GO:0070171] (biological process) Relationships: is a type of GO:0070168; is a type of regulation of tooth mineralization [GO:0070170]; negatively regulates tooth mineralization [GO:0034505] Definition: Any process that stops, prevents, or reduces the frequency, rate or extent of tooth mineralization, the deposition of calcium salts in tooth structures. Sources: GOC:BHF, GOC:mah Subtypes: GO:0070174